{
  "gene_symbol": "MGAT1",
  "gene": "UniProtKB:P26572",
  "term_id": "GO:0006487",
  "term_label": "protein N-linked glycosylation",
  "gene_name": "Alpha-1,3-mannosyl-glycoprotein 2-beta-N-acetylglucosaminyltransferase"
}